positive regulation of L-glutamine biosynthetic process [GO:0062134] (biological process) Relationships: is a type of positive regulation of small molecule metabolic process [GO:0062013]; is a type of GO:0062132; is a type of GO:2000284; positively regulates GO:1901704 Definition: Any process that starts, increases the frequency, rate or extent of L-glutamine biosynthesis. References: PMID:19755423 Sources: GOC:ha